{
  "term_label": "RNA polymerase II cis-regulatory region sequence-specific DNA binding",
  "gene": "UniProtKB:A0A1W2PPM1",
  "gene_symbol": "CPHXL",
  "gene_name": "Cytoplasmic polyadenylated homeobox-like protein",
  "term_id": "GO:0000978"
}